{
  "gene_symbol": "CFAP418",
  "term_label": "photoreceptor cell morphogenesis",
  "term_id": "GO:0008594",
  "gene": "UniProtKB:Q96NL8",
  "gene_name": "Cilia- and flagella-associated protein 418"
}